{
  "gene_symbol": "OSBPL6",
  "gene_name": "Oxysterol-binding protein-related protein 6",
  "term_label": "cholesterol binding",
  "gene": "UniProtKB:Q9BZF3",
  "term_id": "GO:0015485"
}